{
  "term_id": "GO:0090575",
  "term_label": "RNA polymerase II transcription regulator complex",
  "gene_symbol": "E2F5",
  "gene": "UniProtKB:Q15329",
  "gene_name": "Transcription factor E2F5"
}